electroception [GO:0050956] (biological process) References: PMID:10210663 Sources: GOC:ai, Wikipedia:Electroreception Relationships: is a type of sensory perception of electrical stimulus [GO:0050952] Definition: The series of events required for an organism to receive an electrical stimulus, convert it to a molecular signal, and recognize and characterize the signal. Many fish possess an electroception sense; for example, the electric eel uses low voltage pulses of electricity for navigation and prey location. Also known as: electroception sense, electroceptive sense